{
  "gene_name": "Protein TASOR",
  "gene_symbol": "TASOR",
  "term_id": "GO:0003682",
  "gene": "UniProtKB:Q9UK61",
  "term_label": "chromatin binding"
}